{
  "term_id": "GO:0003729",
  "gene_symbol": "SNIP1",
  "gene_name": "Smad nuclear-interacting protein 1",
  "term_label": "mRNA binding",
  "gene": "UniProtKB:Q8TAD8"
}